{
  "gene_symbol": "CTPS1",
  "gene": "UniProtKB:P17812",
  "gene_name": "CTP synthase 1",
  "term_id": "GO:0097268",
  "term_label": "cytoophidium"
}